{
  "gene_name": "DNA damage-inducible transcript 3 protein",
  "term_label": "DNA-binding transcription activator activity, RNA polymerase II-specific",
  "term_id": "GO:0001228",
  "gene": "UniProtKB:P35638",
  "gene_symbol": "DDIT3"
}